promoter-specific chromatin binding [GO:1990841] (MF) Relationships: is_a chromatin binding [GO:0003682] Definition: Binding to a section of chromatin that is associated with gene promoter sequences of DNA. References: PMID:19948729